{
  "gene": "UniProtKB:Q15466",
  "term_id": "GO:0003714",
  "term_label": "transcription corepressor activity",
  "gene_symbol": "NR0B2",
  "gene_name": "Nuclear receptor subfamily 0 group B member 2"
}